{
  "term_label": "synaptic membrane adhesion",
  "gene": "UniProtKB:Q96NI6",
  "gene_name": "Leucine-rich repeat and fibronectin type-III domain-containing protein 5",
  "term_id": "GO:0099560",
  "gene_symbol": "LRFN5"
}